{
  "term_id": "GO:0071035",
  "gene_name": "Exosome complex component RRP43",
  "gene": "UniProtKB:Q96B26",
  "gene_symbol": "EXOSC8",
  "term_label": "nuclear polyadenylation-dependent rRNA catabolic process"
}